{
  "gene_symbol": "BAG5",
  "gene": "UniProtKB:Q9UL15",
  "term_id": "GO:0016020",
  "gene_name": "BAG family molecular chaperone regulator 5",
  "term_label": "membrane"
}